{
  "gene": "UniProtKB:P51617",
  "term_id": "GO:0005737",
  "gene_name": "Interleukin-1 receptor-associated kinase 1",
  "term_label": "cytoplasm",
  "gene_symbol": "IRAK1"
}